gibberellic acid homeostasis [GO:0010336] (BP) References: PMID:17194763 Relationships: is a type of GO:0055088 Definition: Any biological process involved in the maintenance of an internal steady state of gibberellic acid; may involve transport, biosynthesis, catabolism or conjugation. Also known as: gibberellin homeostasis